kynurenine-glyoxylate transaminase activity [GO:0047315] (molecular function) Also known as: kynurenine-glyoxylate aminotransferase activity, L-kynurenine:glyoxylate aminotransferase (cyclizing), kynurenine--glyoxylate aminotransferase activity Sources: EC:2.6.1.63, RHEA:19249 Definition: Catalysis of the reaction: L-kynurenine + glyoxylate = 4-(2-aminophenyl)-2,4-dioxobutanoate + glycine. Relationships: is a type of transaminase activity [GO:0008483]